{
  "gene_symbol": "NDN",
  "gene": "UniProtKB:Q99608",
  "term_id": "GO:0000122",
  "term_label": "negative regulation of transcription by RNA polymerase II",
  "gene_name": "Necdin"
}